{
  "gene_name": "Myosin light chain 4",
  "gene_symbol": "MYL4",
  "term_label": "myosin II complex",
  "term_id": "GO:0016460",
  "gene": "UniProtKB:P12829"
}